{
  "gene": "UniProtKB:Q5JPE7",
  "gene_name": "BOS complex subunit NOMO2",
  "term_label": "Unknown biological process",
  "gene_symbol": "NOMO2",
  "term_id": "UNKNOWN:0002"
}